{
  "term_id": "GO:0007288",
  "term_label": "sperm axoneme assembly",
  "gene": "UniProtKB:Q5JU67",
  "gene_name": "Cilia- and flagella-associated protein 157",
  "gene_symbol": "CFAP157"
}